{
  "term_id": "GO:0008544",
  "gene_name": "Sciellin",
  "gene_symbol": "SCEL",
  "gene": "UniProtKB:O95171",
  "term_label": "epidermis development"
}